{
  "gene_symbol": "PTPN18",
  "term_label": "protein tyrosine phosphatase activity",
  "gene": "UniProtKB:Q99952",
  "term_id": "GO:0004725",
  "gene_name": "Tyrosine-protein phosphatase non-receptor type 18"
}